{
  "gene_name": "Mucosal addressin cell adhesion molecule 1",
  "term_id": "GO:0002687",
  "term_label": "positive regulation of leukocyte migration",
  "gene": "UniProtKB:Q13477",
  "gene_symbol": "MADCAM1"
}